{
  "term_id": "GO:0005681",
  "gene_symbol": "TXNL4B",
  "gene_name": "Thioredoxin-like protein 4B",
  "term_label": "spliceosomal complex",
  "gene": "UniProtKB:Q9NX01"
}